{
  "gene": "UniProtKB:Q96NK8",
  "term_label": "E-box binding",
  "term_id": "GO:0070888",
  "gene_symbol": "NEUROD6",
  "gene_name": "Neurogenic differentiation factor 6"
}